{
  "gene": "UniProtKB:Q9Y4R8",
  "term_label": "telomeric DNA binding",
  "term_id": "GO:0042162",
  "gene_symbol": "TELO2",
  "gene_name": "Telomere length regulation protein TEL2 homolog"
}